{
  "term_label": "chromatin remodeling",
  "gene_symbol": "FBXL19",
  "gene": "UniProtKB:Q6PCT2",
  "term_id": "GO:0006338",
  "gene_name": "F-box_LRR-repeat protein 19"
}